{
  "gene": "UniProtKB:Q8NDH2",
  "gene_name": "Leucine-rich repeat transmembrane protein CCDC168",
  "term_id": "UNKNOWN:0002",
  "gene_symbol": "CCDC168",
  "term_label": "Unknown biological process"
}